{
  "term_id": "UNKNOWN:0001",
  "term_label": "Unknown molecular function",
  "gene": "UniProtKB:P09758",
  "gene_name": "Tumor-associated calcium signal transducer 2",
  "gene_symbol": "TACSTD2"
}